cis-Golgi-derived vesicle fusion with Golgi medial cisterna membrane [GO:1990691] (biological process) Relationships: is_a Golgi vesicle fusion to target membrane [GO:0048210]; is a type of vesicle fusion with Golgi apparatus [GO:0048280]; is part of inter-Golgi cisterna vesicle-mediated transport [GO:0048219] References: PMID:16038056, PMID:24119662 Sources: GOC:bhm Also known as: cis-Golgi-derived vesicle fusion with medial-Golgi cisterna membrane Definition: The joining of the lipid bilayer membrane around a cis-Golgi-derived vesicle to the lipid bilayer membrane around the medial-Golgi cisterna. Vesicles are involved in anterograde transport.